{
  "term_label": "negative regulation of transcription by RNA polymerase II",
  "term_id": "GO:0000122",
  "gene": "UniProtKB:P0C7X2",
  "gene_symbol": "ZNF688",
  "gene_name": "Zinc finger protein 688"
}